{
  "term_id": "UNKNOWN:0001",
  "gene_name": "NACHT, LRR and PYD domains-containing protein 10",
  "gene": "UniProtKB:Q86W26",
  "gene_symbol": "NLRP10",
  "term_label": "Unknown molecular function"
}